{
  "gene": "UniProtKB:Q8NH02",
  "term_id": "GO:0005886",
  "term_label": "plasma membrane",
  "gene_symbol": "OR2T29",
  "gene_name": "Olfactory receptor 2T29"
}